{
  "gene_symbol": "KRT24",
  "term_id": "GO:0030855",
  "gene_name": "Keratin, type I cytoskeletal 24",
  "term_label": "epithelial cell differentiation",
  "gene": "UniProtKB:Q2M2I5"
}